{
  "gene_name": "Sphingosine 1-phosphate receptor 1",
  "term_label": "sphingosine-1-phosphate receptor activity",
  "gene": "UniProtKB:P21453",
  "gene_symbol": "S1PR1",
  "term_id": "GO:0038036"
}